{
  "gene_symbol": "ADCY8",
  "term_label": "adenylate cyclase activity",
  "term_id": "GO:0004016",
  "gene": "UniProtKB:P40145",
  "gene_name": "Adenylate cyclase type 8"
}